{
  "gene_symbol": "DAOA",
  "gene_name": "D-amino acid oxidase activator",
  "term_id": "GO:0005794",
  "gene": "UniProtKB:P59103",
  "term_label": "Golgi apparatus"
}